{
  "gene": "UniProtKB:Q96AH0",
  "gene_symbol": "NABP1",
  "term_label": "SOSS complex",
  "term_id": "GO:0070876",
  "gene_name": "SOSS complex subunit B2"
}